{
  "term_label": "mitochondrion",
  "gene": "UniProtKB:Q9BX68",
  "gene_symbol": "HINT2",
  "gene_name": "Adenosine 5'-monophosphoramidase HINT2",
  "term_id": "GO:0005739"
}